{
  "gene_name": "Calcium_calmodulin-dependent protein kinase type IV",
  "gene": "UniProtKB:Q16566",
  "term_id": "GO:0035556",
  "term_label": "intracellular signal transduction",
  "gene_symbol": "CAMK4"
}